{
  "gene_symbol": "Q9BTK2",
  "gene": "UniProtKB:Q9BTK2",
  "term_label": "Unknown cellular component",
  "term_id": "UNKNOWN:0003",
  "gene_name": "Putative uncharacterized protein LOC642776"
}